{
  "gene_symbol": "TRIP11",
  "term_label": "Golgi organization",
  "term_id": "GO:0007030",
  "gene": "UniProtKB:Q15643",
  "gene_name": "Thyroid receptor-interacting protein 11"
}